{
  "gene": "UniProtKB:Q7Z6E9",
  "gene_symbol": "RBBP6",
  "term_label": "ubiquitin-dependent protein catabolic process",
  "term_id": "GO:0006511",
  "gene_name": "E3 ubiquitin-protein ligase RBBP6"
}